metal ion transport [GO:0030001] (biological process) Sources: GOC:ai Subtypes: transition metal ion transport [GO:0000041], GO:0006813, sodium ion transport [GO:0006814], calcium ion transport [GO:0006816], lithium ion transport [GO:0010351], aluminum cation transport [GO:0015690], GO:0015692, GO:0015693 Regulation: RO_0002211 by regulation of metal ion transport [GO:0010959] Definition: The directed movement of metal ions, any metal ion with an electric charge, into, out of or within a cell, or between cells, by means of some agent such as a transporter or pore. Relationships: is a type of monoatomic cation transport [GO:0006812] Also known as: divalent metal ion export, divalent metal ion transport, heavy metal ion transport, metal ion export